{
  "gene_name": "Paired mesoderm homeobox protein 2A",
  "term_label": "DNA-binding transcription factor activity, RNA polymerase II-specific",
  "gene_symbol": "PHOX2A",
  "term_id": "GO:0000981",
  "gene": "UniProtKB:O14813"
}